{
  "gene_name": "Protein LDOC1",
  "term_label": "Unknown biological process",
  "gene_symbol": "LDOC1",
  "term_id": "UNKNOWN:0002",
  "gene": "UniProtKB:O95751"
}